larynx morphogenesis [GO:0120223] (biological process) References: PMID:28177282 Sources: GOC:krc Relationships: is a type of animal organ morphogenesis [GO:0009887]; is part of GO:0120224 Definition: The process in which the larynx is generated and organized. The larynx is a continuation of the pharynx that is involved in breathing, sound production, and protecting the trachea against food aspiration. Also known as: laryngeal morphogenesis